positive regulation of establishment or maintenance of cell polarity regulating cell shape [GO:2000771] (biological process) Definition: Any process that activates or increases the frequency, rate or extent of establishment or maintenance of cell polarity regulating cell shape. Sources: GOC:mah Relationships: is a type of GO:0048522; is a type of regulation of establishment or maintenance of cell polarity regulating cell shape [GO:2000769]; positively regulates establishment or maintenance of cell polarity regulating cell shape [GO:0071963] Subtypes: positive regulation of establishment or maintenance of bipolar cell polarity regulating cell shape [GO:2000247], GO:2000784